{
  "gene_symbol": "TERF2",
  "gene_name": "Telomeric repeat-binding factor 2",
  "term_label": "G-rich strand telomeric DNA binding",
  "term_id": "GO:0098505",
  "gene": "UniProtKB:Q15554"
}